{
  "term_id": "UNKNOWN:0003",
  "gene_name": "Small ribosomal subunit protein eS6",
  "gene": "UniProtKB:P62753",
  "gene_symbol": "RPS6",
  "term_label": "Unknown cellular component"
}